{
  "term_id": "GO:0004181",
  "term_label": "metallocarboxypeptidase activity",
  "gene_name": "Carboxypeptidase A5",
  "gene": "UniProtKB:Q8WXQ8",
  "gene_symbol": "CPA5"
}